{
  "gene_symbol": "SPAG6",
  "term_label": "acrosomal vesicle",
  "gene": "UniProtKB:O75602",
  "term_id": "GO:0001669",
  "gene_name": "Sperm-associated antigen 6"
}